{
  "gene_name": "Endoplasmic reticulum chaperone BiP",
  "gene": "UniProtKB:P11021",
  "term_id": "GO:0042026",
  "term_label": "protein refolding",
  "gene_symbol": "HSPA5"
}